{
  "gene_name": "NADP-dependent malic enzyme, mitochondrial",
  "gene": "UniProtKB:Q16798",
  "term_id": "GO:0005739",
  "gene_symbol": "ME3",
  "term_label": "mitochondrion"
}